{
  "gene_symbol": "EXT1",
  "gene_name": "Exostosin-1",
  "term_id": "GO:0008375",
  "term_label": "acetylglucosaminyltransferase activity",
  "gene": "UniProtKB:Q16394"
}